{
  "gene_symbol": "SAMSN1",
  "gene": "UniProtKB:Q9NSI8",
  "gene_name": "SAM domain-containing protein SAMSN-1",
  "term_label": "nucleus",
  "term_id": "GO:0005634"
}